{
  "gene": "UniProtKB:Q6PCB7",
  "gene_name": "Long-chain fatty acid transport protein 1",
  "term_id": "GO:0044539",
  "term_label": "long-chain fatty acid import into cell",
  "gene_symbol": "SLC27A1"
}